left tetrad [GO:0097566] (cellular component) Relationships: is a type of cellular anatomical structure [GO:0110165]; BFO_0000050 cell projection [GO:0042995]; has part left lateral basal body pair [GO:0097562]; has part left middle basal body pair [GO:0097563] Note: Due to the asymmetric nature of the Giardia trophozoite, this term is defined spatially as the trophozoite is viewed from the dorsal side, with the two nuclei dorsal to the ventral disc, and the ventral disc toward the anterior. Definition: Set of four basal bodies found in Giardia species (trophozoite stage). It comprises the left lateral basal body pair and the left middle basal body pair (i.e. the anterior, ventral, caudal and posteriolateral basal bodies located to the right of the left nucleus of the trophozoite when viewed dorsally). References: PMID:16607022, PMID:5961344 Sources: GOC:giardia, ISBN:9780124260207